threonine-type endopeptidase activity [GO:0004298] (molecular function) Relationships: is a type of endopeptidase activity [GO:0004175]; is a type of threonine-type peptidase activity [GO:0070003] Also known as: threonine endopeptidase activity, large multicatalytic protease, lens neutral proteinase, multicatalytic proteinase, multicatalytic proteinase (complex), proteasome endopeptidase complex, tricorn protease, tricorn proteinase, 26S protease, MCP, alkaline protease, ingensin, multicatalytic endopeptidase complex, prosome Sources: GOC:mah, https://www.ebi.ac.uk/merops/about/glossary.shtml#CATTYPE, https://www.ebi.ac.uk/merops/about/glossary.shtml#ENDOPEPTIDASE Definition: Catalysis of the hydrolysis of internal peptide bonds in a polypeptide chain by a mechanism in which the hydroxyl group of a threonine residue at the active center acts as a nucleophile.